{
  "gene": "UniProtKB:Q53S08",
  "gene_symbol": "RAB6D",
  "term_label": "endomembrane system",
  "term_id": "GO:0012505",
  "gene_name": "Ras-related protein Rab-6D"
}